response to yeast [GO:0001878] (biological process) Subtypes: GO:0001879 Relationships: is a type of response to fungus [GO:0009620] References: PMID:14707091 Note: defined as response to Saccharomycotina (true yeasts). This excludes fission yeast. Definition: Any process that results in a change in state or activity of a cell or an organism (in terms of movement, secretion, enzyme production, gene expression, etc.) as a result of a stimulus from a yeast species.